cellubrevin-VAMP4-endobrevin-syntaxin-6 complex [GO:0070066] (cellular component) Definition: A SNARE complex that contains cellubrevin (VAMP3), VAMP4, endobrevin (VAMP8), and syntaxin 6 (or orthologs thereof). Also known as: SNARE complex (Vamp3, Vamp4, Vam8, Stx6), Vamp3-Vamp4-Vam8-Stx6 complex References: PMID:11839770 Relationships: is a type of SNARE complex [GO:0031201]